{
  "gene_name": "Dual specificity protein phosphatase CDC14A",
  "term_label": "protein serine/threonine phosphatase activity",
  "term_id": "GO:0004722",
  "gene": "UniProtKB:Q9UNH5",
  "gene_symbol": "CDC14A"
}